{
  "term_label": "Unknown molecular function",
  "term_id": "UNKNOWN:0001",
  "gene_symbol": "LPXN",
  "gene_name": "Leupaxin",
  "gene": "UniProtKB:O60711"
}